heme A biosynthetic process [GO:0006784] (biological process) Definition: The chemical reactions and pathways resulting in the formation of heme A, a derivative of heme found in cytochrome aa3. References: PMID:11788607 Sources: GOC:ai Also known as: haem A biosynthesis, haem A biosynthetic process, heme A anabolism, heme A biosynthesis, heme A formation, heme A synthesis Relationships: is a type of heme biosynthetic process [GO:0006783]